{
  "term_id": "GO:0005886",
  "gene_symbol": "OSCAR",
  "gene": "UniProtKB:Q8IYS5",
  "term_label": "plasma membrane",
  "gene_name": "Osteoclast-associated immunoglobulin-like receptor"
}